positive regulation of transmission of nerve impulse [GO:0051971] (biological process) Sources: GOC:ai Definition: Any process that activates, maintains or increases the frequency, rate or extent of transmission of a nerve impulse, the sequential electrochemical polarization and depolarization that travels across the membrane of a neuron in response to stimulation. Subtypes: positive regulation of neuronal action potential [GO:1904457] Also known as: positive regulation of conduction of nerve impulse, up regulation of transmission of nerve impulse, up-regulation of transmission of nerve impulse, upregulation of transmission of nerve impulse, activation of transmission of nerve impulse, stimulation of transmission of nerve impulse Relationships: is a type of positive regulation of cell communication [GO:0010647]; is a type of positive regulation of nervous system process [GO:0031646]; is a type of regulation of transmission of nerve impulse [GO:0051969]; positively regulates transmission of nerve impulse [GO:0019226]